{
  "term_id": "GO:0003725",
  "gene_name": "Interleukin enhancer-binding factor 3",
  "term_label": "double-stranded RNA binding",
  "gene": "UniProtKB:Q12906",
  "gene_symbol": "ILF3"
}